poly(C) RNA binding [GO:0017130] (molecular function) Relationships: is a type of poly-pyrimidine tract binding [GO:0008187] Definition: Binding to a sequence of cytosine residues in an RNA molecule. Sources: GOC:mah Also known as: poly(C) binding, poly(rC) binding